DNA polymerase III, beta sliding clamp processivity factor complex [GO:0044775] (cellular component) Sources: GOC:jl, UniProt:O73947 Relationships: is a type of DNA polymerase processivity factor complex [GO:0044796]; is part of DNA polymerase III complex [GO:0009360] Definition: A subcomplex of the DNA polymerase III holoenzyme which is responsible for tethering the catalytic subunit of DNA polymerase to DNA during high-speed replication. The complex is homodimeric in prokaryotes, and homotrimeric in other species.